negative regulation of type III interferon production [GO:0034345] (biological process) References: PMID:15546383, PMID:16734557 Sources: GOC:add, ISBN:0126896631 Note: Note that IL-28A, IL-28B, and IL-29 are types of interferon-lambda. Relationships: is a type of GO:0001818; is a type of regulation of type III interferon production [GO:0034344]; negatively regulates type III interferon production [GO:0034343] Also known as: down regulation of type III interferon production, down-regulation of type III interferon production, downregulation of type III interferon production, negative regulation of type III IFN production, inhibition of type III interferon production Definition: Any process that stops, prevents, or reduces the frequency, rate, or extent of type III interferon production. Interferon lambda is the only member of the type III interferon found so far.